{
  "gene": "UniProtKB:Q9UIC8",
  "term_id": "GO:0090266",
  "gene_name": "Leucine carboxyl methyltransferase 1",
  "term_label": "regulation of mitotic cell cycle spindle assembly checkpoint",
  "gene_symbol": "LCMT1"
}